{
  "gene": "UniProtKB:O75339",
  "gene_symbol": "CILP",
  "gene_name": "Cartilage intermediate layer protein 1",
  "term_label": "Unknown molecular function",
  "term_id": "UNKNOWN:0001"
}